positive regulation of monodictyphenone biosynthetic process [GO:1900845] (biological process) Relationships: is a type of positive regulation of small molecule metabolic process [GO:0062013]; is a type of GO:1900378; is a type of regulation of monodictyphenone biosynthetic process [GO:1900843]; positively regulates monodictyphenone biosynthetic process [GO:1900815] Sources: GOC:TermGenie, GOC:di Also known as: upregulation of monodictyphenone biosynthetic process Definition: Any process that activates or increases the frequency, rate or extent of monodictyphenone biosynthetic process.